{
  "term_id": "UNKNOWN:0001",
  "gene_symbol": "MCRIP2",
  "gene": "UniProtKB:Q9BUT9",
  "gene_name": "MAPK regulated corepressor interacting protein 2",
  "term_label": "Unknown molecular function"
}